{
  "gene_symbol": "FAM89B",
  "term_label": "positive regulation of cell migration",
  "gene_name": "Leucine repeat adapter protein 25",
  "gene": "UniProtKB:Q8N5H3",
  "term_id": "GO:0030335"
}